{
  "gene_symbol": "PSMB10",
  "term_label": "proteasome core complex, beta-subunit complex",
  "gene_name": "Proteasome subunit beta type-10",
  "gene": "UniProtKB:P40306",
  "term_id": "GO:0019774"
}